{
  "term_label": "neuron projection development",
  "gene_name": "Mesencephalic astrocyte-derived neurotrophic factor",
  "gene": "UniProtKB:P55145",
  "gene_symbol": "MANF",
  "term_id": "GO:0031175"
}